{
  "gene_name": "Tubulin gamma-1 chain",
  "term_label": "microtubule nucleator activity",
  "gene": "UniProtKB:P23258",
  "term_id": "GO:0140490",
  "gene_symbol": "TUBG1"
}